{
  "term_id": "GO:0042470",
  "gene": "UniProtKB:P40967",
  "term_label": "melanosome",
  "gene_symbol": "PMEL",
  "gene_name": "Melanocyte protein PMEL"
}